{
  "term_label": "Unknown molecular function",
  "gene_symbol": "SAMD12",
  "gene": "UniProtKB:Q8N8I0",
  "term_id": "UNKNOWN:0001",
  "gene_name": "Sterile alpha motif domain-containing protein 12"
}